sneeze reflex [GO:0160023] (biological process) Also known as: sternutation Relationships: is a type of reflex [GO:0060004] Definition: A reflex process that expels air forcibly from the mouth and nose in an explosive, spasmodic involuntary action resulting chiefly from irritation of the nasal mucous membrane. References: PMID:34133943 Sources: https://www.thefreedictionary.com/sneeze